{
  "term_id": "GO:0098609",
  "gene_name": "Catenin delta-2",
  "term_label": "cell-cell adhesion",
  "gene_symbol": "CTNND2",
  "gene": "UniProtKB:Q9UQB3"
}